{
  "gene_name": "Enolase 4",
  "term_label": "phosphopyruvate hydratase activity",
  "gene": "UniProtKB:A6NNW6",
  "term_id": "GO:0004634",
  "gene_symbol": "ENO4"
}